{
  "gene": "UniProtKB:Q9H8H0",
  "term_label": "nucleolus",
  "gene_name": "Nucleolar protein 11",
  "term_id": "GO:0005730",
  "gene_symbol": "NOL11"
}